{
  "term_id": "GO:0005737",
  "term_label": "cytoplasm",
  "gene": "UniProtKB:P78560",
  "gene_symbol": "CRADD",
  "gene_name": "Death domain-containing protein CRADD"
}